{
  "gene": "UniProtKB:Q16696",
  "term_id": "GO:0008392",
  "gene_symbol": "CYP2A13",
  "gene_name": "Cytochrome P450 2A13",
  "term_label": "arachidonate epoxygenase activity"
}